{
  "term_label": "nucleolus",
  "gene_name": "Glutamate-rich WD repeat-containing protein 1",
  "term_id": "GO:0005730",
  "gene": "UniProtKB:Q9BQ67",
  "gene_symbol": "GRWD1"
}